{
  "gene_name": "Spastin",
  "term_label": "cytoplasm",
  "gene_symbol": "SPAST",
  "term_id": "GO:0005737",
  "gene": "UniProtKB:Q9UBP0"
}